{
  "term_id": "GO:0051087",
  "term_label": "protein-folding chaperone binding",
  "gene_name": "DnaJ homolog subfamily C member 3",
  "gene": "UniProtKB:Q13217",
  "gene_symbol": "DNAJC3"
}